{
  "term_label": "regulation of transcription by RNA polymerase II",
  "gene_name": "Nuclear receptor subfamily 6 group A member 1",
  "term_id": "GO:0006357",
  "gene": "UniProtKB:Q15406",
  "gene_symbol": "NR6A1"
}